polyprenol metabolic process [GO:0016093] (biological process) References: PMID:11108713 Subtypes: polyprenol biosynthetic process [GO:0016094], GO:0016095, farnesol metabolic process [GO:0016487] Also known as: polyprenol metabolism Relationships: is a type of alcohol metabolic process [GO:0006066]; is a type of isoprenoid metabolic process [GO:0006720] Definition: The chemical reactions and pathways involving polyprenols, prenols with more than 4 isoprenoid residues, which may be all-trans, or a mixture of cis and trans.